{
  "gene": "UniProtKB:Q9Y2J4",
  "gene_name": "Angiomotin-like protein 2",
  "term_id": "GO:0030036",
  "gene_symbol": "AMOTL2",
  "term_label": "actin cytoskeleton organization"
}